glutamate synthase activity [GO:0015930] (molecular function) Sources: GOC:curators Definition: Catalysis of the formation of L-glutamine and 2-oxoglutarate from L-glutamate, using NADH, NADPH or ferredoxin as hydrogen acceptors. Relationships: is a type of oxidoreductase activity, acting on the CH-NH2 group of donors [GO:0016638] Subtypes: GO:0004355, glutamate synthase (NADH) activity [GO:0016040], glutamate synthase (ferredoxin) activity [GO:0016041]